{
  "gene": "UniProtKB:Q96HH4",
  "gene_symbol": "TMEM169",
  "term_label": "Unknown biological process",
  "gene_name": "Transmembrane protein 169",
  "term_id": "UNKNOWN:0002"
}